{
  "term_id": "GO:0000978",
  "gene_symbol": "MEF2B",
  "term_label": "RNA polymerase II cis-regulatory region sequence-specific DNA binding",
  "gene_name": "Myocyte-specific enhancer factor 2B",
  "gene": "UniProtKB:Q02080"
}